{
  "gene_name": "Zinc finger CCCH-type antiviral protein 1",
  "gene_symbol": "ZC3HAV1",
  "gene": "UniProtKB:Q7Z2W4",
  "term_label": "Unknown molecular function",
  "term_id": "UNKNOWN:0001"
}